{
  "gene_name": "Excitatory amino acid transporter 3",
  "gene": "UniProtKB:P43005",
  "term_label": "glutamate:sodium symporter activity",
  "term_id": "GO:0015501",
  "gene_symbol": "SLC1A1"
}